purine deoxyribonucleotide catabolic process [GO:0009155] (biological process) Sources: GOC:go_curators, ISBN:0198506732 Relationships: is a type of purine nucleotide catabolic process [GO:0006195]; is a type of purine deoxyribonucleotide metabolic process [GO:0009151]; is a type of deoxyribonucleotide catabolic process [GO:0009264]; is a type of deoxyribose phosphate catabolic process [GO:0046386] Also known as: purine deoxyribonucleotide breakdown, purine deoxyribonucleotide catabolism, purine deoxyribonucleotide degradation Definition: The chemical reactions and pathways resulting in the breakdown of purine deoxyribonucleotide, a compound consisting of deoxyribonucleoside (a purine base linked to a deoxyribose sugar) esterified with a phosphate group at either the 3' or 5'-hydroxyl group of the sugar. Subtypes: GO:0006203, dITP catabolic process [GO:0035863], dGMP catabolic process [GO:0046055], dADP catabolic process [GO:0046057], GO:0046059, dATP catabolic process [GO:0046061], GO:0046067